{
  "term_label": "gap junction channel activity involved in AV node cell-bundle of His cell electrical coupling",
  "gene": "UniProtKB:Q8N144",
  "gene_name": "Gap junction delta-3 protein",
  "term_id": "GO:0086077",
  "gene_symbol": "GJD3"
}